{
  "term_id": "GO:0036064",
  "term_label": "ciliary basal body",
  "gene_symbol": "CEP78",
  "gene": "UniProtKB:Q5JTW2",
  "gene_name": "Centrosomal protein of 78 kDa"
}